CNTFR-CLCF1 complex [GO:0097059] (cellular component) Definition: A protein complex that is composed of two soluble ciliary neurotrophic factor receptor alpha subunits (product of the CNTFR gene) and two molecules of cardiotrophin-like cytokine factor 1 (product of the CLCF1 gene). The complex is secreted into the extracellular space. References: PMID:11285233 Sources: GOC:BHF Relationships: is_a protein-containing complex [GO:0032991]; is part of GO:0005576 Also known as: sCNTFR-CLC complex